{
  "gene_name": "A-kinase-interacting protein 1",
  "gene_symbol": "AKIP1",
  "term_id": "GO:0005654",
  "gene": "UniProtKB:Q9NQ31",
  "term_label": "nucleoplasm"
}